metal cation:proton antiporter activity [GO:0051139] (molecular function) Sources: GOC:mlg Definition: Enables the transfer of a solute or solutes from one side of a membrane to the other according to the reaction: metal ion(in) + H+(out) = metal ion(out) + H+(in). Also known as: metal ion:hydrogen antiporter activity, metal ion:proton antiporter activity Relationships: is a type of proton transmembrane transporter activity [GO:0015078]; is a type of GO:0140828 Subtypes: GO:0010348, manganese:proton antiporter activity [GO:0010486], calcium:proton antiporter activity [GO:0015369], sodium:proton antiporter activity [GO:0015385], GO:0015386, zinc:proton antiporter activity [GO:0140826]